{
  "term_id": "GO:0007052",
  "gene": "UniProtKB:Q9H3R5",
  "gene_symbol": "CENPH",
  "term_label": "mitotic spindle organization",
  "gene_name": "Centromere protein H"
}